Cul8-RING ubiquitin ligase complex [GO:0035361] (cellular component) References: PMID:20139071 Sources: GOC:krc Relationships: is a type of cullin-RING ubiquitin ligase complex [GO:0031461] Definition: A ubiquitin ligase complex in which a cullin from the Cul8 subfamily and a RING domain protein form the catalytic core. In S. cerevisiae, Mms1p acts as the adaptor protein and substrate specificity is conferred by any of a number of different proteins.